{
  "gene": "UniProtKB:Q8NCR3",
  "term_id": "UNKNOWN:0001",
  "gene_symbol": "MFI",
  "term_label": "Unknown molecular function",
  "gene_name": "Protein MFI"
}